{
  "gene": "UniProtKB:Q6ZN01",
  "gene_name": "MEF2-activating motif and SAP domain-containing transcriptional regulator",
  "term_label": "regulation of transcription by RNA polymerase II",
  "gene_symbol": "MAMSTR",
  "term_id": "GO:0006357"
}